positive regulation of neosartoricin biosynthetic process [GO:1902055] (biological process) Definition: Any process that activates or increases the frequency, rate or extent of neosartoricin biosynthetic process. References: PMID:23368997 Sources: GOC:TermGenie, GOC:di Relationships: is a type of positive regulation of polyketide biosynthetic process [GO:1900734]; is a type of regulation of neosartoricin biosynthetic process [GO:1902053]; is a type of positive regulation of alcohol biosynthetic process [GO:1902932]; RO_0002213 GO:1902050 Also known as: activation of neosartoricin anabolism, activation of neosartoricin biosynthesis, activation of neosartoricin formation, activation of neosartoricin synthesis, positive regulation of neosartoricin anabolism, positive regulation of neosartoricin biosynthesis, positive regulation of neosartoricin formation, positive regulation of neosartoricin synthesis, up regulation of neosartoricin anabolism, up regulation of neosartoricin biosynthesis, up regulation of neosartoricin biosynthetic process, up regulation of neosartoricin formation, up regulation of neosartoricin synthesis, up-regulation of neosartoricin anabolism, up-regulation of neosartoricin biosynthesis, up-regulation of neosartoricin biosynthetic process, up-regulation of neosartoricin formation, up-regulation of neosartoricin synthesis, upregulation of neosartoricin anabolism, upregulation of neosartoricin biosynthesis, upregulation of neosartoricin biosynthetic process, upregulation of neosartoricin formation, upregulation of neosartoricin synthesis, activation of neosartoricin biosynthetic process